{
  "gene_name": "Sister chromatid cohesion protein PDS5 homolog A",
  "term_label": "cohesin unloader activity",
  "gene": "UniProtKB:Q29RF7",
  "term_id": "GO:0140670",
  "gene_symbol": "PDS5A"
}